{
  "gene_name": "Achaete-scute homolog 1",
  "term_id": "GO:0030182",
  "gene_symbol": "ASCL1",
  "gene": "UniProtKB:P50553",
  "term_label": "neuron differentiation"
}